{
  "gene_symbol": "PODNL1",
  "gene": "UniProtKB:Q6PEZ8",
  "term_id": "UNKNOWN:0002",
  "gene_name": "Podocan-like protein 1",
  "term_label": "Unknown biological process"
}